{
  "gene": "UniProtKB:Q7RTY0",
  "term_label": "plasma membrane",
  "gene_symbol": "SLC16A13",
  "gene_name": "Monocarboxylate transporter 13",
  "term_id": "GO:0005886"
}